{
  "gene_name": "Beta-1,4 N-acetylgalactosaminyltransferase 2",
  "term_label": "UDP-N-acetylglucosamine metabolic process",
  "term_id": "GO:0006047",
  "gene_symbol": "B4GALNT2",
  "gene": "UniProtKB:Q8NHY0"
}